{
  "gene_name": "Small ribosomal subunit protein eS26",
  "gene": "UniProtKB:P62854",
  "gene_symbol": "RPS26",
  "term_id": "GO:0003735",
  "term_label": "structural constituent of ribosome"
}